{
  "gene_name": "IQ motif and SEC7 domain-containing protein 3",
  "term_label": "postsynaptic density membrane",
  "gene_symbol": "IQSEC3",
  "gene": "UniProtKB:Q9UPP2",
  "term_id": "GO:0098839"
}